regulation of iron-sulfur cluster assembly [GO:1903329] (biological process) Subtypes: GO:1900487, regulation of [4Fe-4S] cluster assembly [GO:1900491], regulation of iron-sulfur-molybdenum cofactor assembly [GO:1900506], negative regulation of iron-sulfur cluster assembly [GO:1903330], GO:1903331 Sources: GOC:TermGenie, GOC:vw, GO_REF:0000058 Definition: Any process that modulates the frequency, rate or extent of iron-sulfur cluster assembly. Relationships: is a type of GO:0044087; is a type of regulation of cellular component organization [GO:0051128]; regulates iron-sulfur cluster assembly [GO:0016226]